{
  "gene_symbol": "GNAO1",
  "term_label": "corticotropin-releasing hormone receptor 1 binding",
  "term_id": "GO:0051430",
  "gene_name": "Guanine nucleotide-binding protein G(o) subunit alpha",
  "gene": "UniProtKB:P09471"
}